{
  "term_label": "neuromuscular junction",
  "gene": "UniProtKB:Q9UPQ7",
  "term_id": "GO:0031594",
  "gene_name": "E3 ubiquitin-protein ligase PDZRN3",
  "gene_symbol": "PDZRN3"
}